ecdysteroid-phosphate phosphatase activity [GO:0102531] (molecular function) References: PMID:12721294 Sources: MetaCyc:RXN-14734 Also known as: ecdysone-phosphate phosphatase activity Definition: Catalysis of the reaction: H2O + an ecdysteroid 22-phosphate = phosphate + an ecdysteroid. Also has activity towards other ecdysteriod phosphates including 20-hydroxyecdysone 22-phosphate (20E22P) and 2-deoxyecdysone 22-phosphate (2dE22P). Relationships: is a type of phosphatase activity [GO:0016791]